{
  "gene_symbol": "UTS2B",
  "term_label": "regulation of blood pressure",
  "gene_name": "Urotensin-2B",
  "gene": "UniProtKB:Q765I0",
  "term_id": "GO:0008217"
}